negative regulation of protein localization [GO:1903828] (biological process) Relationships: is a type of regulation of protein localization [GO:0032880]; is a type of negative regulation of biological process [GO:0048519]; negatively regulates GO:0008104 Also known as: down regulation of cellular protein localisation, down regulation of cellular protein localization, down-regulation of cellular protein localisation, down-regulation of cellular protein localization, downregulation of cellular protein localisation, downregulation of cellular protein localization, negative regulation of cellular protein localisation, negative regulation of cellular protein localization, inhibition of cellular protein localisation, inhibition of cellular protein localization Subtypes: GO:0051224, negative regulation of protein localization to cell division site involved in mitotic actomyosin contractile ring assembly [GO:0110084], negative regulation of protein localization to chromatin [GO:0120186], negative regulation of protein localization to lysosome [GO:0150033], negative regulation of protein localization to cell-cell junction [GO:0150119], negative regulation of protein localization to nucleus [GO:1900181], GO:1902364, negative regulation of protein localization to microtubule [GO:1902817], negative regulation of protein localization to cell tip [GO:1903067], negative regulation of protein localization to cilium [GO:1903565], negative regulation of protein localization to cell periphery [GO:1904376], negative regulation of protein localization to centrosome [GO:1904780], negative regulation of asymmetric protein localization involved in cell fate determination [GO:1904786], negative regulation of protein localization to chromosome, telomeric region [GO:1904815], negative regulation of protein localization to phagocytic vesicle [GO:1905170], negative regulation of protein localization to kinetochore [GO:1905341], negative regulation of protein localization to presynapse [GO:1905385], GO:1905476, negative regulation of protein localization to endoplasmic reticulum [GO:1905551], negative regulation of protein localization to endosome [GO:1905667], negative regulation of protein localization to cell leading edge [GO:1905872], negative regulation of protein localization to cell surface [GO:2000009] Sources: GOC:TermGenie, GOC:vw, GO_REF:0000058 Definition: Any process that stops, prevents or reduces the frequency, rate or extent of a protein localization.